{
  "gene_symbol": "TNFRSF1A",
  "gene": "UniProtKB:P19438",
  "term_id": "GO:0005031",
  "term_label": "tumor necrosis factor receptor activity",
  "gene_name": "Tumor necrosis factor receptor superfamily member 1A"
}